{
  "term_label": "SCF ubiquitin ligase complex",
  "gene_symbol": "FBXL21P",
  "term_id": "GO:0019005",
  "gene_name": "Putative F-box_LRR-repeat protein 21",
  "gene": "UniProtKB:Q9UKT6"
}